katanin complex [GO:0008352] (CC) Relationships: is a type of microtubule associated complex [GO:0005875]; is part of microtubule organizing center [GO:0005815] Note: Consider also annotating to the molecular function term 'microtubule-severing ATPase activity ; GO:0008568'. Definition: A complex possessing an activity that couples ATP hydrolysis to the severing of microtubules; usually a heterodimer comprising a catalytic subunit (often 60kDa) and a regulatory subunit (often 80 kDa). References: PMID:10910766